{
  "gene": "UniProtKB:Q9HCN4",
  "gene_name": "GPN-loop GTPase 1",
  "gene_symbol": "GPN1",
  "term_id": "UNKNOWN:0003",
  "term_label": "Unknown cellular component"
}